DNA-binding transcription repressor activity, RNA polymerase II-specific [GO:0001227] (molecular function) Also known as: RNA polymerase II transcription regulatory region sequence-specific DNA binding transcription factor activity involved in negative regulation of transcription, transcriptional repressor activity, RNA polymerase II transcription regulatory region sequence-specific DNA binding, RNA polymerase II core promoter proximal region sequence-specific DNA binding transcription factor activity involved in negative regulation of transcription, RNA polymerase II distal enhancer sequence-specific DNA-binding transcription factor activity involved in negative regulation of transcription, RNA polymerase II transcriptional repressor activity, metal ion regulated core promoter proximal region sequence-specific binding, RNA polymerase II transcriptional repressor activity, metal ion regulated proximal promoter sequence-specific DNA binding, distal enhancer DNA-binding transcription repressor activity, RNA polymerase II-specific, metal ion regulated core promoter proximal region sequence-specific DNA binding RNA polymerase II transcription factor activity involved in negative regulation of transcription, metal ion regulated sequence-specific DNA binding transcription factor activity involved in negative regulation of transcription, proximal promoter DNA-binding transcription repressor activity, RNA polymerase II-specific, sequence-specific distal enhancer binding RNA polymerase II transcription factor activity involved in negative regulation of transcription, transcriptional repressor activity, RNA polymerase II distal enhancer sequence-specific binding, transcriptional repressor activity, RNA polymerase II proximal promoter sequence-specific DNA binding, transcriptional repressor activity, metal ion regulated sequence-specific DNA binding Definition: A DNA-binding transcription factor activity that represses or decreases the transcription of specific gene sets transcribed by RNA polymerase II. Sources: GOC:txnOH-2018 Relationships: is a type of GO:0000981; is a type of DNA-binding transcription repressor activity [GO:0001217]; is part of negative regulation of transcription by RNA polymerase II [GO:0000122] Note: For usage guidance, see comment in GO:0003700 ; DNA-binding transcription factor activity.